{
  "term_id": "GO:0000139",
  "gene": "UniProtKB:O00391",
  "gene_symbol": "QSOX1",
  "term_label": "Golgi membrane",
  "gene_name": "Sulfhydryl oxidase 1"
}